positive regulation of formation of growth cone in injured axon [GO:1905944] (biological process) Relationships: is a type of positive regulation of sprouting of injured axon [GO:0048687]; is a type of regulation of formation of growth cone in injured axon [GO:1905942]; positively regulates formation of growth cone in injured axon [GO:0048689] Definition: Any process that activates or increases the frequency, rate or extent of formation of growth cone in injured axon. References: PMID:19737525 Sources: GOC:TermGenie, GO_REF:0000058 Also known as: up regulation of formation of growth cone in injured axon, up-regulation of formation of growth cone in injured axon, upregulation of formation of growth cone in injured axon, activation of formation of growth cone in injured axon